{
  "term_label": "alpha-beta T cell receptor complex",
  "gene_name": "T cell receptor beta constant 1",
  "term_id": "GO:0042105",
  "gene_symbol": "TRBC1",
  "gene": "UniProtKB:P01850"
}